regulation of cytokine production involved in immune response [GO:0002718] (biological process) Definition: Any process that modulates the frequency, rate, or extent of cytokine production that contributes to an immune response. Sources: GOC:add Subtypes: GO:0002719, positive regulation of cytokine production involved in immune response [GO:0002720], regulation of B cell cytokine production [GO:0002721], regulation of T cell cytokine production [GO:0002724], regulation of natural killer cell cytokine production [GO:0002727], regulation of dendritic cell cytokine production [GO:0002730], regulation of macrophage cytokine production [GO:0010935], regulation of mast cell cytokine production [GO:0032763] Relationships: is a type of GO:0001817; is a type of regulation of production of molecular mediator of immune response [GO:0002700]; regulates cytokine production involved in immune response [GO:0002367] Also known as: regulation of cytokine biosynthetic process involved in immune response, regulation of cytokine secretion involved in immune response, regulation of cytokine production during immune response